male somatic sex determination [GO:0019102] (biological process) Relationships: is a type of GO:0018993; is a type of male sex determination [GO:0030238] Definition: The determination of sex and sexual phenotypes in a male organism's soma. Sources: GOC:mah